{
  "gene_symbol": "TLR6",
  "gene_name": "Toll-like receptor 6",
  "term_id": "GO:0005886",
  "gene": "UniProtKB:Q9Y2C9",
  "term_label": "plasma membrane"
}